periplasmic space organization [GO:0043580] (biological process) Definition: A process that is carried out at the cellular level which results in the assembly, arrangement of constituent parts, or disassembly of the periplasmic space, the region between the inner (cytoplasmic) and outer membrane in Gram-negative bacteria, or the inner membrane and cell wall in fungi. Also known as: periplasmic space organisation, periplasmic space organization and biogenesis Relationships: is a type of cellular component organization [GO:0016043] Sources: GOC:dph, GOC:jl, GOC:mah